{
  "term_id": "GO:0003723",
  "gene": "UniProtKB:Q86U38",
  "gene_name": "Nucleolar protein 9",
  "gene_symbol": "NOP9",
  "term_label": "RNA binding"
}